{
  "gene": "UniProtKB:Q14684",
  "term_label": "chromosome",
  "gene_symbol": "RRP1B",
  "gene_name": "Ribosomal RNA processing protein 1 homolog B",
  "term_id": "GO:0005694"
}